{
  "term_label": "Unknown biological process",
  "gene_name": "Protein FAM156A_FAM156B",
  "term_id": "UNKNOWN:0002",
  "gene_symbol": "FAM156B",
  "gene": "UniProtKB:Q8NDB6"
}